negative regulation of hemostasis [GO:1900047] (biological process) Also known as: down regulation of hemostasis, down-regulation of hemostasis, downregulation of hemostasis, inhibition of hemostasis Subtypes: GO:0030195 Relationships: is a type of negative regulation of biological process [GO:0048519]; is a type of GO:1900046; negatively regulates GO:0007599 Sources: GOC:TermGenie Definition: Any process that stops, prevents or reduces the frequency, rate or extent of hemostasis.